{
  "gene_name": "Ubiquitin carboxyl-terminal hydrolase 17",
  "gene_symbol": "USP17L2",
  "term_label": "regulation of apoptotic process",
  "gene": "UniProtKB:Q6R6M4",
  "term_id": "GO:0042981"
}